mRNA m(6)A methyltransferase activity [GO:0001734] (molecular function) Definition: Catalysis of the reaction: an adenosine in mRNA + S-adenosyl-L-methionine = an N(6)-methyladenosine in mRNA + H+ + S-adenosyl-L-homocysteine. This activity is the methylation of adenines in mRNA with the consensus sequence RRACH, where R is a purine, and H is C, A, or U. Relationships: is a type of mRNA methyltransferase activity [GO:0008174] Also known as: mRNA (N6-adenosine)-methyltransferase activity Sources: EC:2.1.1.348, GOC:hjd